{
  "term_id": "GO:0006682",
  "term_label": "galactosylceramide biosynthetic process",
  "gene_name": "2-hydroxyacylsphingosine 1-beta-galactosyltransferase",
  "gene_symbol": "UGT8",
  "gene": "UniProtKB:Q16880"
}